{
  "gene_symbol": "CACNG8",
  "gene_name": "Voltage-dependent calcium channel gamma-8 subunit",
  "term_id": "GO:0098839",
  "gene": "UniProtKB:Q8WXS5",
  "term_label": "postsynaptic density membrane"
}